positive regulation of high voltage-gated calcium channel activity [GO:1901843] (biological process) Relationships: is a type of GO:1901387; positively regulates high voltage-gated calcium channel activity [GO:0008331] Also known as: activation of high voltage gated calcium channel activity, activation of high voltage-dependent calcium channel activity, positive regulation of high voltage gated calcium channel activity, positive regulation of high voltage-dependent calcium channel activity, up regulation of high voltage gated calcium channel activity, up regulation of high voltage-dependent calcium channel activity, up regulation of high voltage-gated calcium channel activity, up-regulation of high voltage gated calcium channel activity, up-regulation of high voltage-dependent calcium channel activity, up-regulation of high voltage-gated calcium channel activity, upregulation of high voltage gated calcium channel activity, upregulation of high voltage-dependent calcium channel activity, upregulation of high voltage-gated calcium channel activity, activation of high voltage-gated calcium channel activity References: PMID:12754254 Sources: GOC:BHF, GOC:TermGenie, GOC:rl Definition: Any process that activates or increases the frequency, rate or extent of high voltage-gated calcium channel activity.